{
  "term_id": "GO:0005814",
  "gene_symbol": "RTTN",
  "term_label": "centriole",
  "gene_name": "Rotatin",
  "gene": "UniProtKB:Q86VV8"
}